{
  "term_label": "plasma membrane",
  "gene": "UniProtKB:Q9BZR6",
  "gene_symbol": "RTN4R",
  "gene_name": "Reticulon-4 receptor",
  "term_id": "GO:0005886"
}